monensin A biosynthetic process [GO:1901730] (biological process) Definition: The chemical reactions and pathways resulting in the formation of monensin A. Relationships: is a type of alcohol biosynthetic process [GO:0046165]; is a type of carboxylic acid biosynthetic process [GO:0046394] Also known as: monensin A anabolism, monensin A biosynthesis, monensin A formation, monensin A synthesis, monensin anabolism, monensin biosynthesis, monensin formation, monensin synthesis Sources: GOC:TermGenie, GOC:yaf, UniPathway:UPA00178